{
  "term_label": "Notch signaling pathway",
  "gene": "UniProtKB:Q14469",
  "gene_name": "Transcription factor HES-1",
  "term_id": "GO:0007219",
  "gene_symbol": "HES1"
}